{
  "term_id": "GO:0033691",
  "gene_symbol": "SIGLEC5",
  "gene_name": "Sialic acid-binding Ig-like lectin 5",
  "term_label": "sialic acid binding",
  "gene": "UniProtKB:O15389"
}